{
  "gene_symbol": "KRTAP4-5",
  "term_label": "hair cycle",
  "gene": "UniProtKB:Q9BYR2",
  "term_id": "GO:0042633",
  "gene_name": "Keratin-associated protein 4-5"
}